{
  "term_label": "glycosylphosphatidylinositol phospholipase D activity",
  "gene": "UniProtKB:P80108",
  "gene_symbol": "GPLD1",
  "term_id": "GO:0004621",
  "gene_name": "Phosphatidylinositol-glycan-specific phospholipase D"
}